{
  "term_label": "Unknown molecular function",
  "term_id": "UNKNOWN:0001",
  "gene_name": "Integrator complex subunit 9",
  "gene": "UniProtKB:Q9NV88",
  "gene_symbol": "INTS9"
}